regulation of cyclodextrin catabolic process [GO:2000957] (biological process) Also known as: regulation of cyclodextrin catabolism Relationships: is a type of regulation of polysaccharide metabolic process [GO:0032881]; is a type of regulation of carbohydrate catabolic process [GO:0043470]; regulates cyclodextrin catabolic process [GO:2000901] Sources: GOC:mengo_curators Subtypes: negative regulation of cyclodextrin catabolic process [GO:2000958], positive regulation of cyclodextrin catabolic process [GO:2000959] Definition: Any process that modulates the frequency, rate or extent of cyclodextrin catabolic process.